anthranilate synthase complex [GO:0005950] (cellular component) References: PMID:4886290 Definition: A heterotetrameric enzyme complex made up of two components I and two components II. Catalyzes the formation of anthranilate, pyruvate and L-glutamate from chorismate and L-glutamine. Relationships: is a type of catalytic complex [GO:1902494]; is part of GO:0005737